{
  "term_id": "GO:0000146",
  "gene_symbol": "MYO1C",
  "term_label": "microfilament motor activity",
  "gene": "UniProtKB:O00159",
  "gene_name": "Unconventional myosin-Ic"
}